{
  "gene_symbol": "HSF4",
  "term_label": "Unknown biological process",
  "gene_name": "Heat shock factor protein 4",
  "term_id": "UNKNOWN:0002",
  "gene": "UniProtKB:Q9ULV5"
}